{
  "gene_name": "Target of rapamycin complex subunit LST8",
  "term_label": "TORC1 complex",
  "gene": "UniProtKB:Q9BVC4",
  "gene_symbol": "MLST8",
  "term_id": "GO:0031931"
}